{
  "gene": "UniProtKB:P04003",
  "gene_name": "C4b-binding protein alpha chain",
  "term_id": "GO:0005615",
  "gene_symbol": "C4BPA",
  "term_label": "extracellular space"
}